{
  "gene": "UniProtKB:P23280",
  "term_id": "GO:0004089",
  "gene_name": "Carbonic anhydrase 6",
  "term_label": "carbonate dehydratase activity",
  "gene_symbol": "CA6"
}